{
  "term_label": "regulation of protein secretion",
  "gene_name": "Inactive rhomboid protein 2",
  "gene_symbol": "RHBDF2",
  "term_id": "GO:0050708",
  "gene": "UniProtKB:Q6PJF5"
}